{
  "term_label": "Unknown biological process",
  "term_id": "UNKNOWN:0002",
  "gene": "UniProtKB:A0A075B6U8",
  "gene_name": "T cell receptor alpha joining 12 (Fragment)",
  "gene_symbol": "TRAJ12"
}